response to alkane [GO:1902778] (biological process) Subtypes: response to hexane [GO:1901499], GO:1902779, response to nonane [GO:1902780], response to decane [GO:1902782], response to undecane [GO:1902784], response to dodecane [GO:1902786], response to isooctane [GO:1902788] Also known as: process resulting in tolerance to alkane References: PMID:22958739, PMID:23826995 Sources: GOC:TermGenie, GOC:mengo_curators, GO_REF:0000071 Relationships: is a type of GO:0042221 Definition: Any process that results in a change in state or activity of a cell or an organism (in terms of movement, secretion, enzyme production, gene expression, etc.) as a result of an alkane stimulus.